proanthocyanidin biosynthetic process [GO:0010023] (biological process) Also known as: proanthocyanidin anabolism, proanthocyanidin biosynthesis, proanthocyanidin formation, proanthocyanidin synthesis Definition: The chemical reactions and pathways resulting in the formation of proanthocyanidin. Sources: GOC:lm Regulation: regulated by regulation of proanthocyanidin biosynthetic process [GO:2000029] Relationships: is a type of phenylpropanoid biosynthetic process [GO:0009699]; is a type of GO:0046189